{
  "gene": "UniProtKB:P20132",
  "term_id": "GO:0003941",
  "term_label": "L-serine ammonia-lyase activity",
  "gene_symbol": "SDS",
  "gene_name": "L-serine dehydratase_L-threonine deaminase"
}